{
  "term_label": "nucleus",
  "gene_symbol": "TGIF1",
  "gene": "UniProtKB:Q15583",
  "gene_name": "Homeobox protein TGIF1",
  "term_id": "GO:0005634"
}